{
  "gene": "UniProtKB:Q13485",
  "gene_name": "Mothers against decapentaplegic homolog 4",
  "gene_symbol": "SMAD4",
  "term_label": "anatomical structure morphogenesis",
  "term_id": "GO:0009653"
}